DNA 5'-adenosine monophosphate hydrolase activity [GO:0033699] (molecular function) Definition: Catalysis of the reactions: a 5'-end adenosine-5'-diphospho-5'-2'-deoxyribonucleoside-DNA + H2O = a 5'-end 5'-phospho-2'-deoxyribonucleoside-DNA + AMP + 2 H+; and: a 5'-end adenosine-5'-diphospho-5'-ribonucleoside-2'-deoxyribonucleotide-DNA + H2O = a 5'-end 5'-phospho-ribonucleoside-2'-deoxyribonucleotide-DNA + AMP + 2 H+. Nucleophilic release of a covalently linked adenylate residue from a DNA strand, leaving a 5' phosphate terminus. References: PMID:16547001, PMID:17276982 Sources: EC:3.6.1.71, GOC:mah Also known as: DNA adenylate hydrolysis activity, DNA 5'-adenylate hydrolase activity, AMP-removal activity, DNA de-adenylation, DNA deadenylation Relationships: is a type of pyrophosphatase activity [GO:0016462]